{
  "gene": "UniProtKB:P52732",
  "gene_symbol": "KIF11",
  "gene_name": "Kinesin-like protein KIF11",
  "term_id": "GO:0051231",
  "term_label": "spindle elongation"
}